{
  "term_label": "glycerol transmembrane transport",
  "gene_symbol": "AQP9",
  "term_id": "GO:0015793",
  "gene_name": "Aquaporin-9",
  "gene": "UniProtKB:O43315"
}